{
  "gene_name": "Zinc finger protein 90 homolog",
  "term_label": "nucleus",
  "term_id": "GO:0005634",
  "gene_symbol": "ZFP90",
  "gene": "UniProtKB:Q8TF47"
}